{
  "gene_symbol": "Q8NA96",
  "gene": "UniProtKB:Q8NA96",
  "gene_name": "Putative uncharacterized protein FLJ35723",
  "term_id": "UNKNOWN:0003",
  "term_label": "Unknown cellular component"
}